{
  "term_label": "extracellular space",
  "term_id": "GO:0005615",
  "gene_name": "Platelet-derived growth factor C",
  "gene": "UniProtKB:Q9NRA1",
  "gene_symbol": "PDGFC"
}